{
  "gene_name": "Ubiquinol-cytochrome-c reductase complex assembly factor 6",
  "gene_symbol": "UQCC6",
  "term_id": "GO:0034551",
  "term_label": "mitochondrial respiratory chain complex III assembly",
  "gene": "UniProtKB:Q69YU5"
}